{
  "gene_symbol": "CFC1B",
  "gene_name": "Cryptic family protein 1B",
  "term_label": "extracellular region",
  "term_id": "GO:0005576",
  "gene": "UniProtKB:P0CG36"
}